{
  "gene_symbol": "SP3",
  "term_label": "DNA-binding transcription factor activity, RNA polymerase II-specific",
  "term_id": "GO:0000981",
  "gene_name": "Transcription factor Sp3",
  "gene": "UniProtKB:Q02447"
}